{
  "gene_symbol": "ERVFRD-1",
  "gene": "UniProtKB:P60508",
  "term_id": "UNKNOWN:0003",
  "term_label": "Unknown cellular component",
  "gene_name": "Syncytin-2"
}